{
  "gene_name": "Gamma-aminobutyric acid receptor-associated protein-like 3",
  "term_label": "autophagosome membrane",
  "gene_symbol": "GABARAPL3",
  "gene": "UniProtKB:Q9BY60",
  "term_id": "GO:0000421"
}